aralkylamine dehydrogenase (azurin) activity [GO:0030059] (molecular function) Also known as: aralkylamine:(azurin) oxidoreductase (deaminating) activity, aromatic amine dehydrogenase (azurin) activity Relationships: is a type of oxidoreductase activity, acting on the CH-NH2 group of donors, with a copper protein as acceptor [GO:0052877] References: PMID:10506161 Sources: RHEA:47796 Definition: Catalysis of the reaction: an aralkylamine + H2O + 2 oxidized [azurin] = an aromatic aldehyde + 2 H+ + NH4+ + 2 reduced [azurin].